{
  "term_id": "UNKNOWN:0003",
  "gene_symbol": "OPRPN",
  "gene_name": "Opiorphin prepropeptide",
  "gene": "UniProtKB:Q99935",
  "term_label": "Unknown cellular component"
}